proximal/distal pattern formation [GO:0009954] (biological process) Sources: GOC:dph, GOC:go_curators, GOC:isa_complete Also known as: proximal/distal pattern specification Subtypes: proximal/distal pattern formation, imaginal disc [GO:0007449], leaf proximal/distal pattern formation [GO:0010589], maintenance of imaginal disc-derived wing hair orientation [GO:0035321], proximal/distal pattern formation involved in nephron development [GO:0072047] Definition: The regionalization process in which specific areas of cell differentiation are determined along a proximal/distal axis. The proximal/distal axis is defined by a line that runs from main body (proximal end) of an organism outward (distal end). Relationships: is a type of regionalization [GO:0003002]